high mobility group box 1 binding [GO:0070379] (molecular function) Definition: Binding to high mobility group box 1 (HMBGB1). References: PMID:18431461 Sources: GOC:add Also known as: HMGB1 binding Relationships: is a type of cytokine binding [GO:0019955]